[citrate (pro-3S)-lyase] ligase activity [GO:0008771] (molecular function) Relationships: is a type of acid-thiol ligase activity [GO:0016878] Definition: Catalysis of the reaction: ATP + acetate + (citrate (pro-3S)-lyase) (thiol form) = AMP + diphosphate + (citrate (pro-3S)-lyase) (acetyl form). Also known as: acetate:citrate-(pro-3S)-lyase(thiol-form) ligase (AMP-forming), acetate: SH-acyl-carrier-protein enzyme ligase (AMP), acetate:HS-citrate lyase ligase activity, citrate (pro-3S)-lyase ligase activity, citrate lyase ligase activity, citrate lyase synthetase activity Sources: EC:6.2.1.22